positive regulation of extrinsic apoptotic signaling pathway in absence of ligand [GO:2001241] (biological process) Relationships: is a type of positive regulation of extrinsic apoptotic signaling pathway [GO:2001238]; is a type of regulation of extrinsic apoptotic signaling pathway in absence of ligand [GO:2001239]; positively regulates extrinsic apoptotic signaling pathway in absence of ligand [GO:0097192] Also known as: positive regulation of extrinsic apoptotic signalling pathway in absence of ligand, positive regulation of extrinsic apoptosis in absence of ligand, positive regulation of dependence receptor signaling pathway Sources: GOC:mtg_apoptosis Definition: Any process that activates or increases the frequency, rate or extent of extrinsic apoptotic signaling pathway in absence of ligand.